{
  "gene": "UniProtKB:O00716",
  "term_label": "RNA polymerase II cis-regulatory region sequence-specific DNA binding",
  "term_id": "GO:0000978",
  "gene_name": "Transcription factor E2F3",
  "gene_symbol": "E2F3"
}